{
  "term_id": "GO:0016567",
  "gene_name": "BTB_POZ domain-containing adapter for CUL3-mediated RhoA degradation protein 2",
  "term_label": "protein ubiquitination",
  "gene": "UniProtKB:Q13829",
  "gene_symbol": "TNFAIP1"
}